purine deoxyribonucleoside triphosphate catabolic process [GO:0009217] (biological process) Also known as: purine deoxyribonucleoside triphosphate breakdown, purine deoxyribonucleoside triphosphate catabolism, purine deoxyribonucleoside triphosphate degradation Subtypes: dGTP catabolic process [GO:0006203], dITP catabolic process [GO:0035863], dATP catabolic process [GO:0046061] Sources: GOC:go_curators, ISBN:0198506732 Definition: The chemical reactions and pathways resulting in the breakdown of purine deoxyribonucleoside triphosphate, a compound consisting of a purine base linked to a deoxyribose sugar esterified with triphosphate on the sugar. Relationships: is a type of GO:0009146; is a type of deoxyribonucleoside triphosphate catabolic process [GO:0009204]; is a type of purine deoxyribonucleoside triphosphate metabolic process [GO:0009215]